{
  "gene": "UniProtKB:Q14676",
  "gene_symbol": "MDC1",
  "term_id": "GO:0006974",
  "gene_name": "Mediator of DNA damage checkpoint protein 1",
  "term_label": "DNA damage response"
}